{
  "term_label": "UDP-sugar diphosphatase activity",
  "term_id": "GO:0008768",
  "gene_name": "Uridine diphosphate glucose pyrophosphatase NUDT14",
  "gene": "UniProtKB:O95848",
  "gene_symbol": "NUDT14"
}